alpha-amyrin synthase activity [GO:0042561] (molecular function) Definition: Catalysis of the reaction: (S)-2,3-epoxysqualene = alpha-amyrin. This reaction is a cyclization and rearrangement of (S)-2,3-epoxysqualene (2,3-oxidosqualene) into alpha-amyrin. References: PMID:10848960 Sources: GOC:jl, MetaCyc:RXN-8434 Relationships: is a type of oxidosqualene cyclase activity [GO:0031559]